{
  "gene": "UniProtKB:Q15319",
  "term_id": "UNKNOWN:0003",
  "gene_name": "POU domain, class 4, transcription factor 3",
  "term_label": "Unknown cellular component",
  "gene_symbol": "POU4F3"
}